{
  "term_label": "Unknown molecular function",
  "gene": "UniProtKB:Q5VYV7",
  "gene_symbol": "SLX4IP",
  "gene_name": "Protein SLX4IP",
  "term_id": "UNKNOWN:0001"
}